{
  "gene": "UniProtKB:P43166",
  "term_label": "cytoplasm",
  "gene_name": "Carbonic anhydrase 7",
  "term_id": "GO:0005737",
  "gene_symbol": "CA7"
}